{
  "gene_symbol": "AKNAD1",
  "gene": "UniProtKB:Q5T1N1",
  "term_id": "UNKNOWN:0003",
  "term_label": "Unknown cellular component",
  "gene_name": "Protein AKNAD1"
}